{
  "term_id": "GO:0040037",
  "gene_name": "Protein sprouty homolog 3",
  "gene": "UniProtKB:O43610",
  "term_label": "negative regulation of fibroblast growth factor receptor signaling pathway",
  "gene_symbol": "SPRY3"
}